{
  "gene_symbol": "TNS2",
  "gene": "UniProtKB:Q63HR2",
  "term_label": "focal adhesion",
  "gene_name": "Tensin-2",
  "term_id": "GO:0005925"
}